{
  "term_id": "UNKNOWN:0001",
  "gene_symbol": "FNDC1",
  "gene": "UniProtKB:Q4ZHG4",
  "gene_name": "Fibronectin type III domain-containing protein 1",
  "term_label": "Unknown molecular function"
}